glyoxal biosynthetic process [GO:1903191] (biological process) Sources: GOC:PARL, GOC:TermGenie, GOC:bf, GO_REF:0000068 Also known as: glyoxal anabolism, glyoxal biosynthesis, glyoxal formation, glyoxal synthesis Definition: The chemical reactions and pathways resulting in the formation of glyoxal. Relationships: is a type of aldehyde biosynthetic process [GO:0046184]; is a type of glyoxal metabolic process [GO:1903189]